{
  "gene_name": "Gephyrin",
  "gene_symbol": "GPHN",
  "term_label": "cytoplasm",
  "term_id": "GO:0005737",
  "gene": "UniProtKB:Q9NQX3"
}